negative regulation of autophagosome size [GO:0045771] (biological process) Relationships: is a type of regulation of autophagosome size [GO:0016243] Sources: GOC:autophagy, GOC:go_curators Also known as: down regulation of autophagic vacuole size, down-regulation of autophagic vacuole size, downregulation of autophagic vacuole size, negative regulation of autophagic vacuole size, inhibition of autophagic vacuole size Definition: Any process that reduces autophagosome size.